{
  "term_id": "GO:0008090",
  "gene_symbol": "DYNC1H1",
  "term_label": "retrograde axonal transport",
  "gene": "UniProtKB:Q14204",
  "gene_name": "Cytoplasmic dynein 1 heavy chain 1"
}